2-hydroxybiphenyl 3-monooxygenase (NADH) activity [GO:0047544] (molecular function) Definition: Catalysis of the reaction: biphenyl-2-ol + H+ + NADH + O2 = biphenyl-2,3-diol + H2O + NAD+. Also converts 2,2'-dihydroxybiphenyl into 2,2',3-trihydroxy-biphenyl. Also known as: 2-hydroxybiphenyl,NADH:oxygen oxidoreductase (3-hydroxylating) Relationships: is a type of GO:0016709 Sources: EC:1.14.13.44